{
  "gene": "UniProtKB:Q96JJ6",
  "gene_name": "Junctophilin-4",
  "gene_symbol": "JPH4",
  "term_label": "regulation of synaptic plasticity",
  "term_id": "GO:0048167"
}